{
  "term_id": "UNKNOWN:0003",
  "term_label": "Unknown cellular component",
  "gene_name": "Coiled-coil domain-containing protein 103",
  "gene": "UniProtKB:Q8IW40",
  "gene_symbol": "CCDC103"
}